negative regulation of metanephric nephron tubule epithelial cell differentiation [GO:0072308] (biological process) Relationships: is a type of negative regulation of nephron tubule epithelial cell differentiation [GO:0072183]; is a type of regulation of metanephric nephron tubule epithelial cell differentiation [GO:0072307]; negatively regulates GO:0072257 Sources: GOC:mtg_kidney_jan10 Definition: Any process that decreases the frequency, rate or extent of metanephric nephron tubule epithelial cell differentiation.